5(S)-hydroxyperoxy-6E,8Z,11Z,14Z-icosatetraenoic acid binding [GO:0050648] (molecular function) Definition: Binding to 5(S)-hydroxyperoxy-6E,8Z,11Z,14Z-icosatetraenoic acid, a straight-chain fatty acid with twenty carbon atoms and four double bonds. Relationships: is a type of long-chain fatty acid binding [GO:0036041]; is a type of icosanoid binding [GO:0050542]; is a type of GO:1901567 Sources: GOC:ai Also known as: 5(S)-hydroxyperoxy-6E,8Z,11Z,14Z-eicosatetraenoic acid binding